{
  "gene_name": "Pro-adrenomedullin",
  "gene_symbol": "ADM",
  "term_id": "GO:0035809",
  "term_label": "regulation of urine volume",
  "gene": "UniProtKB:P35318"
}